axonemal central apparatus [GO:1990716] (cellular component) Relationships: is a type of cellular anatomical structure [GO:0110165]; is part of axoneme [GO:0005930] Definition: Part of the 9+2 axoneme, that occurs in most motile cilia, consisting of the pair of two single central microtubules and their associated structures which include the central pair projections, the central pair bridges linking the two tubules, and the central pair caps which are attached to the distal or plus ends of the microtubules. References: PMID:21586547, PMID:9295136 Sources: GOC:cilia